{
  "gene": "UniProtKB:O95721",
  "term_id": "GO:0016082",
  "gene_name": "Synaptosomal-associated protein 29",
  "gene_symbol": "SNAP29",
  "term_label": "synaptic vesicle priming"
}